{
  "gene": "UniProtKB:Q96M61",
  "term_label": "nucleus",
  "gene_symbol": "MAGEB18",
  "term_id": "GO:0005634",
  "gene_name": "Melanoma-associated antigen B18"
}